{
  "gene": "UniProtKB:P24903",
  "term_id": "GO:0019373",
  "gene_symbol": "CYP2F1",
  "term_label": "epoxygenase P450 pathway",
  "gene_name": "Cytochrome P450 2F1"
}